tonic smooth muscle contraction [GO:0014820] (biological process) Definition: A process in which force is generated within tonic smooth muscle tissue, resulting in a change in muscle geometry. Force generation involves a chemo-mechanical energy conversion step that is carried out by the actin/myosin complex activity, which generates force through ATP hydrolysis. In the tonic smooth muscle, the muscle contraction occurs without an ordered sarcomeric structure. Tonic smooth muscle contraction occurs as a sustained continuous contraction. Subtypes: artery smooth muscle contraction [GO:0014824], GO:0014847 Relationships: is_a GO:0006939 Sources: GOC:mtg_muscle